{
  "gene_name": "Endogenous retrovirus group K member 7 Pol protein",
  "gene_symbol": "ERVK-7",
  "gene": "UniProtKB:P63135",
  "term_label": "Unknown cellular component",
  "term_id": "UNKNOWN:0003"
}